aleurone grain membrane [GO:0032578] (cellular component) Relationships: is a type of cytoplasmic vesicle membrane [GO:0030659]; is_a bounding membrane of organelle [GO:0098588]; is part of GO:0033095 Definition: The lipid bilayer surrounding an aleurone grain. Sources: GOC:ecd